sweat gland placode formation [GO:0060793] (biological process) Relationships: is a type of ectodermal placode formation [GO:0060788]; is part of sweat gland development [GO:0060792] Definition: The developmental process in which the sweat gland placode forms. An sweat gland placode is a thickening of the ectoderm that will give rise to the sweat gland bud. Sources: GOC:dph, GOC:sdb_2009, GOC:tb